{
  "term_label": "Unknown molecular function",
  "gene_name": "Leucine-rich repeat and calponin homology domain-containing protein 2",
  "gene": "UniProtKB:Q5VUJ6",
  "term_id": "UNKNOWN:0001",
  "gene_symbol": "LRCH2"
}